{
  "term_label": "nucleus",
  "gene_symbol": "MX1",
  "term_id": "GO:0005634",
  "gene": "UniProtKB:P20591",
  "gene_name": "Interferon-induced GTP-binding protein Mx1"
}